negative regulation of vasculature development [GO:1901343] (biological process) Subtypes: negative regulation of vasculature development involved in avascular cornea development in camera-type eye [GO:1901346], negative regulation of blood vessel morphogenesis [GO:2000181] Sources: GOC:TermGenie Definition: Any process that stops, prevents or reduces the frequency, rate or extent of vasculature development. Relationships: is a type of negative regulation of developmental process [GO:0051093]; is a type of GO:0051241; is a type of regulation of vasculature development [GO:1901342]; negatively regulates GO:0001944 Also known as: down regulation of vasculature development, down-regulation of vasculature development, downregulation of vasculature development, inhibition of vasculature development, down regulation of vascular system development, down-regulation of vascular system development, downregulation of vascular system development, inhibition of vascular system development, negative regulation of vascular system development